{
  "gene_symbol": "TAF10",
  "term_label": "promoter-specific chromatin binding",
  "gene_name": "Transcription initiation factor TFIID subunit 10",
  "term_id": "GO:1990841",
  "gene": "UniProtKB:Q12962"
}